{
  "term_id": "GO:0070837",
  "term_label": "dehydroascorbic acid transport",
  "gene_symbol": "SLC2A5",
  "gene": "UniProtKB:P22732",
  "gene_name": "Solute carrier family 2, facilitated glucose transporter member 5"
}